{
  "term_label": "synapse",
  "gene_symbol": "CPEB4",
  "term_id": "GO:0045202",
  "gene": "UniProtKB:Q17RY0",
  "gene_name": "Cytoplasmic polyadenylation element-binding protein 4"
}